UDP-3-O-[(3R)-3-hydroxyacyl]-glucosamine N-acyltransferase activity [GO:0103118] (molecular function) Also known as: UDP-3-O-(R-3-hydroxymyristoyl)-glucosamine N-acyltransferase activity, UDP-3-O-[3-hydroxymyristoyl] glucosamine N-acyltransferase activity Definition: Catalysis of the reaction: a UDP-3-O-[(3R)-3-hydroxyacyl]-alpha-D-glucosamine + a (3R)-hydroxyacyl-[ACP] = a UDP-2-N,3-O-bis[(3R)-3-hydroxyacyl]-alpha-D-glucosamine + holo-[ACP] + H+. Relationships: is a type of acyltransferase activity, transferring groups other than amino-acyl groups [GO:0016747] Sources: RHEA:53836